{
  "gene_name": "Suppressor of fused homolog",
  "term_id": "GO:0005634",
  "gene": "UniProtKB:Q9UMX1",
  "gene_symbol": "SUFU",
  "term_label": "nucleus"
}